{
  "gene_symbol": "RTN4RL2",
  "term_id": "GO:0005886",
  "term_label": "plasma membrane",
  "gene": "UniProtKB:Q86UN3",
  "gene_name": "Reticulon-4 receptor-like 2"
}